{
  "term_label": "cytosol",
  "gene_name": "Importin-7",
  "gene_symbol": "IPO7",
  "term_id": "GO:0005829",
  "gene": "UniProtKB:O95373"
}